{
  "gene_name": "Leukocyte immunoglobulin-like receptor subfamily A member 4",
  "gene": "UniProtKB:P59901",
  "term_id": "GO:0032396",
  "gene_symbol": "LILRA4",
  "term_label": "inhibitory MHC class I receptor activity"
}